{
  "gene_name": "Protein argonaute-1",
  "term_id": "GO:0016442",
  "gene": "UniProtKB:Q9UL18",
  "term_label": "RISC complex",
  "gene_symbol": "AGO1"
}